{
  "gene_name": "Spectrin beta chain, non-erythrocytic 5",
  "gene_symbol": "SPTBN5",
  "term_label": "actin filament binding",
  "term_id": "GO:0051015",
  "gene": "UniProtKB:Q9NRC6"
}